oculomotor nerve formation [GO:0021623] (biological process) Relationships: is a type of cranial nerve formation [GO:0021603]; is part of oculomotor nerve morphogenesis [GO:0021622] Also known as: CN III biosynthesis, CN III formation Sources: GOC:cls, GOC:dgh, GOC:dph, GOC:jid, GO_REF:0000021 Definition: The process that gives rise to the oculomotor nerve. This process pertains to the initial formation of a structure from unspecified parts. This motor nerve innervates all extraocular muscles except the superior oblique and the lateral rectus muscles. The superior division supplies the levator palpebrae superioris and superior rectus muscles. The inferior division supplies the medial rectus, inferior rectus and inferior oblique muscles. This nerve also innervates the striated muscles of the eyelid. Pupillary constriction and lens movement are mediated by this nerve for near vision. In the orbit the inferior division sends branches that enter the ciliary ganglion where they form functional contacts (synapses) with the ganglion cells. The ganglion cells send nerve fibers into the back of the eye where they travel to ultimately innervate the ciliary muscle and the constrictor pupillae muscle.